2-enoate reductase activity [GO:0047540] (molecular function) Definition: Catalysis of the reaction: butanoate + NAD+ = 2-butenoate + NADH + H+. Sources: EC:1.3.1.31, MetaCyc:2-ENOATE-REDUCTASE-RXN Also known as: butanoate:NAD+ delta2-oxidoreductase activity, enoate reductase activity Relationships: is a type of oxidoreductase activity, acting on the CH-CH group of donors, NAD or NADP as acceptor [GO:0016628]